L-glutamate catabolic process to aspartate [GO:0019550] (biological process) Definition: The chemical reactions and pathways resulting in the breakdown of L-glutamate into other compounds, including aspartate. Sources: GOC:go_curators Also known as: glutamate breakdown to aspartate, glutamate degradation to aspartate Relationships: is a type of aspartate metabolic process [GO:0006531]; is a type of L-glutamate catabolic process [GO:0006538]